{
  "gene_symbol": "XKR5",
  "term_id": "GO:0016020",
  "term_label": "membrane",
  "gene_name": "XK-related protein 5",
  "gene": "UniProtKB:Q6UX68"
}